{
  "gene": "UniProtKB:Q9ULT6",
  "gene_symbol": "ZNRF3",
  "term_label": "plasma membrane",
  "gene_name": "E3 ubiquitin-protein ligase ZNRF3",
  "term_id": "GO:0005886"
}